{
  "term_id": "UNKNOWN:0003",
  "term_label": "Unknown cellular component",
  "gene_symbol": "HAGHL",
  "gene_name": "Hydroxyacylglutathione hydrolase-like protein",
  "gene": "UniProtKB:Q6PII5"
}